{
  "term_label": "mitotic spindle midzone assembly",
  "gene_name": "Kinesin-like protein KIF23",
  "gene": "UniProtKB:Q02241",
  "term_id": "GO:0051256",
  "gene_symbol": "KIF23"
}